regulation of toll-like receptor 13 signaling pathway [GO:0034179] (biological process) Definition: Any process that modulates the frequency, rate, or extent of toll-like receptor 13 signaling pathway. References: PMID:16551253, PMID:17328678 Sources: GOC:add Also known as: regulation of TLR13 signaling pathway, regulation of toll-like receptor 13 signalling pathway Relationships: is a type of regulation of cytoplasmic pattern recognition receptor signaling pathway [GO:0039531]; regulates toll-like receptor 13 signaling pathway [GO:0034178] Subtypes: GO:0034180, GO:0034181